{
  "gene_name": "Transcription factor AP-2-alpha",
  "term_id": "GO:0000977",
  "term_label": "RNA polymerase II transcription regulatory region sequence-specific DNA binding",
  "gene": "UniProtKB:P05549",
  "gene_symbol": "TFAP2A"
}